{
  "term_label": "nucleus",
  "gene_name": "Synaptopodin 2-like protein",
  "term_id": "GO:0005634",
  "gene_symbol": "SYNPO2L",
  "gene": "UniProtKB:Q9H987"
}